{
  "term_id": "UNKNOWN:0003",
  "gene_name": "Protein FAM246A",
  "term_label": "Unknown cellular component",
  "gene": "UniProtKB:A0A494C0Y3",
  "gene_symbol": "FAM246A"
}